{
  "term_id": "GO:0000978",
  "gene": "UniProtKB:Q96K62",
  "gene_name": "Zinc finger and BTB domain-containing protein 45",
  "gene_symbol": "ZBTB45",
  "term_label": "RNA polymerase II cis-regulatory region sequence-specific DNA binding"
}